{
  "term_label": "intracellular protein transport",
  "gene_name": "Transmembrane emp24 domain-containing protein 6",
  "gene": "UniProtKB:Q8WW62",
  "term_id": "GO:0006886",
  "gene_symbol": "TMED6"
}